{
  "gene": "UniProtKB:A0A0U1RRN3",
  "gene_symbol": "MISFA",
  "term_label": "Unknown biological process",
  "gene_name": "Mitochondrial sheath formation-associated protein",
  "term_id": "UNKNOWN:0002"
}